{
  "gene_name": "Putative nuclear pore complex-interacting protein family member B2",
  "gene_symbol": "NPIPB2",
  "term_label": "Unknown biological process",
  "gene": "UniProtKB:A6NJ64",
  "term_id": "UNKNOWN:0002"
}